{
  "term_id": "GO:0020037",
  "gene_name": "Cytoglobin",
  "gene": "UniProtKB:Q8WWM9",
  "gene_symbol": "CYGB",
  "term_label": "heme binding"
}